{
  "gene": "UniProtKB:Q9H207",
  "gene_symbol": "OR10A5",
  "term_id": "GO:0004984",
  "term_label": "olfactory receptor activity",
  "gene_name": "Olfactory receptor 10A5"
}